{
  "term_label": "succinyl-CoA metabolic process",
  "gene_name": "Succinate--CoA ligase [ADP-forming] subunit beta, mitochondrial",
  "term_id": "GO:0006104",
  "gene_symbol": "SUCLA2",
  "gene": "UniProtKB:Q9P2R7"
}